{
  "gene": "UniProtKB:P22735",
  "gene_name": "Protein-glutamine gamma-glutamyltransferase K",
  "term_label": "protein-glutamine gamma-glutamyltransferase activity",
  "term_id": "GO:0003810",
  "gene_symbol": "TGM1"
}